{
  "gene": "UniProtKB:P40313",
  "term_label": "serine-type endopeptidase activity",
  "term_id": "GO:0004252",
  "gene_symbol": "CTRL",
  "gene_name": "Chymotrypsin-like protease CTRL-1"
}